{
  "term_id": "UNKNOWN:0001",
  "gene": "UniProtKB:Q9HCB6",
  "gene_symbol": "SPON1",
  "term_label": "Unknown molecular function",
  "gene_name": "Spondin-1"
}